{
  "gene_symbol": "PID1",
  "term_id": "GO:0046325",
  "term_label": "negative regulation of D-glucose import",
  "gene_name": "PTB-containing, cubilin and LRP1-interacting protein",
  "gene": "UniProtKB:Q7Z2X4"
}